{
  "term_id": "GO:0005739",
  "gene_symbol": "CARD19",
  "term_label": "mitochondrion",
  "gene": "UniProtKB:Q96LW7",
  "gene_name": "Caspase recruitment domain-containing protein 19"
}